negative regulation of apoptotic process involved in outflow tract morphogenesis [GO:1902257] (biological process) Also known as: down regulation of apoptotic process involved in outflow tract morphogenesis, down-regulation of apoptotic process involved in outflow tract morphogenesis, downregulation of apoptotic process involved in outflow tract morphogenesis, down regulation of apoptosis involved in outflow tract morphogenesis, down-regulation of apoptosis involved in outflow tract morphogenesis, downregulation of apoptosis involved in outflow tract morphogenesis, inhibition of apoptosis involved in outflow tract morphogenesis, inhibition of apoptotic process involved in outflow tract morphogenesis, negative regulation of apoptosis involved in outflow tract morphogenesis Relationships: is a type of GO:1902256; is a type of negative regulation of apoptotic process involved in morphogenesis [GO:1902338]; negatively regulates apoptotic process involved in outflow tract morphogenesis [GO:0003275] References: PMID:16839542 Sources: GOC:TermGenie, GOC:dph, GOC:mtg_apoptosis Definition: Any process that stops, prevents or reduces the frequency, rate or extent of apoptotic process involved in outflow tract morphogenesis.